apoptotic nuclear changes [GO:0030262] (biological process) Also known as: apoptotic nuclear change Sources: GOC:mah, GOC:mtg_apoptosis Definition: Alterations undergone by nuclei at the molecular and morphological level as part of the execution phase of apoptosis. Relationships: is_a cellular component disassembly involved in execution phase of apoptosis [GO:0006921]